lipoteichoic acid immune receptor activity [GO:0070892] (molecular function) Also known as: lipoteichoic acid receptor activity Definition: Combining with lipoteichoic acid and transmitting the signal to initiate an innate immune response. Relationships: is a type of GO:0038187; has part lipoteichoic acid binding [GO:0070891] References: PMID:14665680 Sources: GOC:add